{
  "gene_name": "Cytoplasmic phosphatidylinositol transfer protein 1",
  "gene_symbol": "PITPNC1",
  "gene": "UniProtKB:Q9UKF7",
  "term_id": "GO:0035091",
  "term_label": "phosphatidylinositol binding"
}